{
  "gene": "UniProtKB:P13631",
  "gene_symbol": "RARG",
  "gene_name": "Retinoic acid receptor gamma",
  "term_label": "RNA polymerase II cis-regulatory region sequence-specific DNA binding",
  "term_id": "GO:0000978"
}